{
  "term_label": "glycine biosynthetic process, by transamination of glyoxylate",
  "gene": "UniProtKB:P21549",
  "term_id": "GO:0019265",
  "gene_symbol": "AGXT",
  "gene_name": "Alanine--glyoxylate aminotransferase"
}